{
  "term_label": "regulation of gene expression",
  "term_id": "GO:0010468",
  "gene_name": "E3 ubiquitin-protein ligase TRIM48",
  "gene_symbol": "TRIM48",
  "gene": "UniProtKB:Q8IWZ4"
}